{
  "gene_symbol": "OPCML",
  "gene": "UniProtKB:Q14982",
  "term_id": "UNKNOWN:0001",
  "gene_name": "Opioid-binding protein_cell adhesion molecule",
  "term_label": "Unknown molecular function"
}